{
  "gene": "UniProtKB:P0DSN7",
  "term_id": "GO:0019814",
  "gene_name": "Probable non-functional immunoglobulinn kappa variable 1D-37",
  "gene_symbol": "IGKV1D-37",
  "term_label": "immunoglobulin complex"
}